chondroblast differentiation [GO:0060591] (biological process) Sources: GOC:dph Relationships: is a type of GO:0030154; is part of cartilage development [GO:0051216] Definition: The process in which a mesenchymal cell, acquires specialized structural and/or functional features of a chondroblast. Differentiation includes the processes involved in commitment of a cell to a chondroblast fate. A chondroblast is a precursor cell to chondrocytes. Also known as: chondrocyte progenitor cell differentiation